phosphatidylglycerophosphatase activity [GO:0008962] (molecular function) Also known as: PGP phosphatase activity, phosphatidylglycerol phosphatase activity, phosphatidylglycerol phosphate phosphatase activity, phosphatidylglycerophosphate phosphohydrolase activity Relationships: is a type of phosphatase activity [GO:0016791] Definition: Catalysis of the reaction: phosphatidylglycerophosphate + H2O = phosphatidylglycerol + phosphate. References: PMID:4292860